{
  "gene": "UniProtKB:Q99758",
  "term_id": "UNKNOWN:0003",
  "gene_name": "Phospholipid-transporting ATPase ABCA3",
  "term_label": "Unknown cellular component",
  "gene_symbol": "ABCA3"
}